{
  "gene_name": "25-hydroxyvitamin D-1 alpha hydroxylase, mitochondrial",
  "gene_symbol": "CYP27B1",
  "term_id": "GO:0005739",
  "term_label": "mitochondrion",
  "gene": "UniProtKB:O15528"
}